{
  "gene_name": "Glutathione S-transferase 3, mitochondrial",
  "term_id": "GO:0005783",
  "gene_symbol": "MGST3",
  "term_label": "endoplasmic reticulum",
  "gene": "UniProtKB:O14880"
}